protein-tetrapyrrole linkage [GO:0017006] (biological process) Definition: The covalent linking of a tetrapyrrole to a protein. Sources: GOC:ai Relationships: is a type of GO:0051604 Subtypes: protein-heme linkage [GO:0017003], protein-bilin linkage [GO:0017007]